{
  "gene": "UniProtKB:Q9H6D8",
  "gene_symbol": "FNDC4",
  "gene_name": "Fibronectin type III domain-containing protein 4",
  "term_id": "UNKNOWN:0003",
  "term_label": "Unknown cellular component"
}